negative regulation of bicellular tight junction assembly [GO:1903347] (biological process) Relationships: is a type of negative regulation of cell junction assembly [GO:1901889]; is a type of regulation of bicellular tight junction assembly [GO:2000810]; negatively regulates bicellular tight junction assembly [GO:0070830] Also known as: down regulation of tight junction assembly, down regulation of tight junction formation, down-regulation of tight junction assembly, down-regulation of tight junction formation, downregulation of tight junction assembly, downregulation of tight junction formation, negative regulation of tight junction formation, inhibition of tight junction assembly, inhibition of tight junction formation Definition: Any process that stops, prevents or reduces the frequency, rate or extent of tight junction assembly. References: PMID:25050009 Sources: GOC:TermGenie, GOC:jz, GO_REF:0000058